regulation of T cell mediated cytotoxicity directed against tumor cell target [GO:0002852] (biological process) Sources: GOC:add Definition: Any process that modulates the frequency, rate, or extent of T cell mediated cytotoxicity directed against a tumor cell target. Subtypes: negative regulation of T cell mediated cytotoxicity directed against tumor cell target [GO:0002853], GO:0002854 Relationships: is a type of regulation of T cell mediated cytotoxicity [GO:0001914]; is a type of regulation of T cell mediated immune response to tumor cell [GO:0002840]; regulates T cell mediated cytotoxicity directed against tumor cell target [GO:0002419]